{
  "gene_name": "Solute carrier family 28 member 3",
  "gene": "UniProtKB:Q9HAS3",
  "term_label": "purine-specific nucleoside:sodium symporter activity",
  "term_id": "GO:0015390",
  "gene_symbol": "SLC28A3"
}